{
  "gene_symbol": "TEP1",
  "gene_name": "Telomerase protein component 1",
  "term_label": "telomerase activity",
  "gene": "UniProtKB:Q99973",
  "term_id": "GO:0003720"
}